{
  "gene_symbol": "PRIMA1",
  "term_id": "UNKNOWN:0001",
  "gene": "UniProtKB:Q86XR5",
  "term_label": "Unknown molecular function",
  "gene_name": "Proline-rich membrane anchor 1"
}